regulation of angioblast cell migration involved in selective angioblast sprouting [GO:0035477] (biological process) Definition: Any process that modulates the frequency, rate or extent of angioblast cell migration involved in selective angioblast sprouting. Relationships: is a type of regulation of anatomical structure morphogenesis [GO:0022603]; is a type of regulation of cell migration [GO:0030334]; is a type of GO:1901342; regulates angioblast cell migration involved in selective angioblast sprouting [GO:0035475] References: PMID:19815777 Sources: GOC:dgh